{
  "gene_name": "TBC1 domain family member 2B",
  "gene": "UniProtKB:Q9UPU7",
  "term_label": "plasma membrane",
  "gene_symbol": "TBC1D2B",
  "term_id": "GO:0005886"
}